{
  "term_label": "Golgi apparatus",
  "term_id": "GO:0005794",
  "gene_symbol": "KIAA0319L",
  "gene": "UniProtKB:Q8IZA0",
  "gene_name": "Dyslexia-associated protein KIAA0319-like protein"
}